{
  "term_label": "adenosine deaminase activity",
  "term_id": "GO:0004000",
  "gene_name": "Adenosine deaminase",
  "gene_symbol": "ADA",
  "gene": "UniProtKB:P00813"
}